{
  "gene_name": "Transcription termination factor 2, mitochondrial",
  "gene_symbol": "MTERF2",
  "gene": "UniProtKB:Q49AM1",
  "term_id": "GO:0003676",
  "term_label": "nucleic acid binding"
}